export across plasma membrane [GO:0140115] (biological process) Definition: The directed movement of some substance from inside of a cell, across the plasma membrane and into the extracellular region. Sources: GOC:pg Also known as: efflux Relationships: is a type of GO:0055085; is a type of export from cell [GO:0140352] Subtypes: auxin export across the plasma membrane [GO:0010315], GO:0010352, GO:0032973, sodium ion export across plasma membrane [GO:0036376], peptide pheromone export by transmembrane transport [GO:0090539], potassium ion export across plasma membrane [GO:0097623], GO:0120029, manganese ion export across plasma membrane [GO:0140048], fluoride export across plasma membrane [GO:0140116], borate export across plasma membrane [GO:0140159], zinc export across plasma membrane [GO:0140882], sulfite export across plasma membrane [GO:0160244], GO:0180029, iron ion export across plasma membrane [GO:1903988], GO:1990034, xenobiotic detoxification by transmembrane export across the plasma membrane [GO:1990961]